{
  "gene": "UniProtKB:Q8IYA7",
  "term_id": "GO:0048468",
  "gene_symbol": "MKX",
  "gene_name": "Homeobox protein Mohawk",
  "term_label": "cell development"
}